{
  "term_id": "UNKNOWN:0001",
  "term_label": "Unknown molecular function",
  "gene_name": "Tetratricopeptide repeat protein 7B",
  "gene_symbol": "TTC7B",
  "gene": "UniProtKB:Q86TV6"
}